{
  "gene": "UniProtKB:Q9NQ69",
  "gene_symbol": "LHX9",
  "gene_name": "LIM_homeobox protein Lhx9",
  "term_id": "GO:0030182",
  "term_label": "neuron differentiation"
}